{
  "term_label": "transcription cis-regulatory region binding",
  "gene_symbol": "ZNF229",
  "gene_name": "Zinc finger protein 229",
  "term_id": "GO:0000976",
  "gene": "UniProtKB:Q9UJW7"
}